{
  "term_id": "UNKNOWN:0001",
  "gene_symbol": "TTC21B",
  "gene_name": "Tetratricopeptide repeat protein 21B",
  "gene": "UniProtKB:Q7Z4L5",
  "term_label": "Unknown molecular function"
}